{
  "term_id": "UNKNOWN:0002",
  "gene_symbol": "SMIM9",
  "gene_name": "Small integral membrane protein 9",
  "gene": "UniProtKB:A6NGZ8",
  "term_label": "Unknown biological process"
}